{
  "gene_name": "cAMP and cAMP-inhibited cGMP 3',5'-cyclic phosphodiesterase 10A",
  "gene": "UniProtKB:Q9Y233",
  "gene_symbol": "PDE10A",
  "term_label": "Unknown cellular component",
  "term_id": "UNKNOWN:0003"
}